establishment or maintenance of monopolar cell polarity regulating cell shape [GO:0061340] (BP) Definition: Any cellular process that results in the specification, formation or maintenance of a monopolar intracellular organization or cell growth patterns that regulate the shape of a cell. Sources: GOC:dph, GOC:vw Relationships: is a type of establishment or maintenance of monopolar cell polarity [GO:0061339]; is a type of GO:0071963